{
  "gene_symbol": "UCP1",
  "term_id": "GO:0009409",
  "gene_name": "Mitochondrial brown fat uncoupling protein 1",
  "gene": "UniProtKB:P25874",
  "term_label": "response to cold"
}